glycerophospholipid acyltransferase (CoA-dependent) activity [GO:0047178] (molecular function) Also known as: 1-organyl-2-acyl-sn-glycero-3-phosphocholine:1-organyl-2-lyso-sn-glycero-3-phosphoethanolamine acyltransferase (CoA-dependent) Sources: EC:2.3.1.148, MetaCyc:2.3.1.148-RXN Relationships: is a type of acyltransferase activity, transferring groups other than amino-acyl groups [GO:0016747] Definition: Catalysis of the reaction: 1-radyl-2-lyso-sn-glycero-3-phosphoethanolamine + 1-radyl-2-acyl-sn-glycero-3-phosphocholine = 1-radyl-2-lyso-sn-glycero-3-phosphocholine + 1-radyl-2-acyl-sn-glycero-3-phosphoethanolamine.